{
  "term_id": "GO:0008284",
  "gene_symbol": "FLT4",
  "term_label": "positive regulation of cell population proliferation",
  "gene": "UniProtKB:P35916",
  "gene_name": "Vascular endothelial growth factor receptor 3"
}